{
  "term_id": "GO:0008157",
  "gene": "UniProtKB:Q9H7J1",
  "term_label": "protein phosphatase 1 binding",
  "gene_symbol": "PPP1R3E",
  "gene_name": "Protein phosphatase 1 regulatory subunit 3E"
}